{
  "gene_symbol": "TRIAP1",
  "term_label": "phospholipid transport",
  "term_id": "GO:0015914",
  "gene": "UniProtKB:O43715",
  "gene_name": "TP53-regulated inhibitor of apoptosis 1"
}